{
  "gene": "UniProtKB:Q8IZP1",
  "term_id": "UNKNOWN:0002",
  "gene_symbol": "TBC1D3",
  "term_label": "Unknown biological process",
  "gene_name": "TBC1 domain family member 3"
}